{
  "term_label": "Unknown cellular component",
  "term_id": "UNKNOWN:0003",
  "gene_name": "Endogenous Bornavirus-like nucleoprotein 2",
  "gene_symbol": "EBLN2",
  "gene": "UniProtKB:Q6P2I7"
}